{
  "gene_symbol": "TCEA1",
  "gene_name": "Transcription elongation factor A protein 1",
  "term_id": "GO:0003711",
  "gene": "UniProtKB:P23193",
  "term_label": "transcription elongation factor activity"
}